{
  "gene_symbol": "TSC22D3",
  "term_id": "GO:0070236",
  "term_label": "negative regulation of activation-induced cell death of T cells",
  "gene_name": "TSC22 domain family protein 3",
  "gene": "UniProtKB:Q99576"
}